{
  "gene_symbol": "CLTC",
  "term_id": "GO:0005819",
  "term_label": "spindle",
  "gene_name": "Clathrin heavy chain 1",
  "gene": "UniProtKB:Q00610"
}